bud dilation [GO:0061137] (biological process) Definition: The process in which a branch bud increases radially. A branch bud is the initial area of outgrowth in the formation of a new branch. Sources: GOC:dph Relationships: is a type of developmental growth involved in morphogenesis [GO:0060560]; is part of morphogenesis of a branching structure [GO:0001763]